{
  "term_id": "GO:0003727",
  "gene": "UniProtKB:Q9BYX4",
  "term_label": "single-stranded RNA binding",
  "gene_symbol": "IFIH1",
  "gene_name": "Interferon-induced helicase C domain-containing protein 1"
}